{
  "term_label": "endoplasmic reticulum",
  "gene_name": "Endoplasmic reticulum-Golgi intermediate compartment protein 2",
  "term_id": "GO:0005783",
  "gene": "UniProtKB:Q96RQ1",
  "gene_symbol": "ERGIC2"
}